microtubule organizing center localization [GO:0061842] (biological process) Definition: Any process in which the microtubule organizing center is transported to, and/or maintained in, a specific location within the cell. References: PMID:21281821 Subtypes: centrosome localization [GO:0051642], spindle pole body localization [GO:0070631] Relationships: is a type of cellular process [GO:0009987]; is a type of localization [GO:0051179] Also known as: MTOC localization, MTOC polarity, microtubule organizing center polarity